{
  "term_id": "GO:0160187",
  "gene": "UniProtKB:Q8N6F1",
  "term_label": "paracellular tight junction channel activity",
  "gene_symbol": "CLDN19",
  "gene_name": "Claudin-19"
}